{
  "term_label": "Unknown molecular function",
  "term_id": "UNKNOWN:0001",
  "gene_name": "Putative gametogenetin-binding protein 1",
  "gene": "UniProtKB:Q5YKI7",
  "gene_symbol": "GGNBP1"
}